4-hydroxymandelate synthase activity [GO:0050585] (MF) Relationships: is a type of oxidoreductase activity, acting on single donors with incorporation of molecular oxygen, incorporation of two atoms of oxygen [GO:0016702] Also known as: 4-hydroxyphenylpyruvate:oxygen oxidoreductase (decarboxylating), 4-hydroxyphenylpyruvate dioxygenase II activity Sources: EC:1.13.11.46, MetaCyc:1.13.11.46-RXN Definition: Catalysis of the reaction: 4-hydroxyphenylpyruvate + O2 = 4-hydroxymandelate + CO2.